positive regulation of platelet rolling [GO:0160018] (biological process) Sources: GOC:sl, GO_REF:0000058 Relationships: is a type of GO:0034116; is a type of GO:0160017; positively regulates platelet rolling [GO:0160015] Definition: Any process that increases the rate, frequency, or extent of platelet rolling.